{
  "gene_name": "Nectin-1",
  "term_id": "GO:0043296",
  "gene": "UniProtKB:Q15223",
  "term_label": "apical junction complex",
  "gene_symbol": "NECTIN1"
}